{
  "gene": "UniProtKB:Q6IN97",
  "gene_symbol": "FRMPD2B",
  "gene_name": "Putative protein FRMPD2-like",
  "term_label": "Unknown biological process",
  "term_id": "UNKNOWN:0002"
}